{
  "term_id": "GO:0006955",
  "gene_symbol": "IGKV2D-40",
  "term_label": "immune response",
  "gene_name": "Immunoglobulin kappa variable 2D-40",
  "gene": "UniProtKB:P01614"
}